{
  "term_label": "olfactory receptor activity",
  "gene_symbol": "OR10J4",
  "gene": "UniProtKB:P0C629",
  "term_id": "GO:0004984",
  "gene_name": "Olfactory receptor 10J4"
}